{
  "gene_name": "Histone chaperone ASF1A",
  "term_label": "histone binding",
  "gene_symbol": "ASF1A",
  "term_id": "GO:0042393",
  "gene": "UniProtKB:Q9Y294"
}